{
  "gene_name": "Dystrophin-related protein 2",
  "term_label": "Unknown molecular function",
  "term_id": "UNKNOWN:0001",
  "gene": "UniProtKB:Q13474",
  "gene_symbol": "DRP2"
}